{
  "gene_symbol": "NUTM2B",
  "gene_name": "NUT family member 2B",
  "gene": "UniProtKB:A6NNL0",
  "term_label": "Unknown cellular component",
  "term_id": "UNKNOWN:0003"
}